regulation of DNA double-strand break processing [GO:1903775] (biological process) References: PMID:25203555 Sources: GOC:TermGenie, GO_REF:0000058 Relationships: is_a GO:0051052; regulates DNA double-strand break processing [GO:0000729] Definition: Any process that modulates the frequency, rate or extent of DNA double-strand break processing.